{
  "gene": "UniProtKB:Q96H86",
  "term_label": "RNA polymerase II transcription regulatory region sequence-specific DNA binding",
  "gene_symbol": "ZNF764",
  "gene_name": "Zinc finger protein 764",
  "term_id": "GO:0000977"
}